{
  "gene_symbol": "CPT1B",
  "term_label": "long-chain fatty acid transport",
  "gene_name": "Carnitine O-palmitoyltransferase 1, muscle isoform",
  "gene": "UniProtKB:Q92523",
  "term_id": "GO:0015909"
}